{
  "term_label": "cilium assembly",
  "gene": "UniProtKB:P61006",
  "gene_symbol": "RAB8A",
  "term_id": "GO:0060271",
  "gene_name": "Ras-related protein Rab-8A"
}